{
  "gene": "UniProtKB:Q6ZN17",
  "term_id": "GO:0003729",
  "gene_symbol": "LIN28B",
  "term_label": "mRNA binding",
  "gene_name": "Protein lin-28 homolog B"
}